G protein-coupled serotonin receptor activity [GO:0004993] (molecular function) Also known as: 5-HT receptor, 5-hydroxytryptamine receptor, G protein coupled serotonin receptor activity, G-protein coupled serotonin receptor activity Sources: GOC:ai Definition: Combining with the biogenic amine serotonin and transmitting the signal across the membrane by activating an associated G-protein. Serotonin (5-hydroxytryptamine) is a neurotransmitter and hormone found in vertebrates and invertebrates. Subtypes: Gi/o-coupled serotonin receptor activity [GO:0001586], GO:0001587 Relationships: is_a G protein-coupled amine receptor activity [GO:0008227]; is part of GO:0098664; has part serotonin binding [GO:0051378]